synaptic vesicle priming [GO:0016082] (biological process) Note: Although this process can occur outside of synaptic transmission, by convention we treat it as a part of synaptic transmission. (dos, pvn, fk synapse project 2015) Relationships: is a type of protein-containing complex assembly [GO:0065003]; is a type of exocytic process [GO:0140029]; BFO_0000050 GO:0016079 Regulation: regulated by regulation of synaptic vesicle priming [GO:0010807]; positively regulated by positive regulation of synaptic vesicle priming [GO:0010808]; negatively regulated by GO:0010809 References: PMID:15217342, PMID:23060190 Sources: GOC:mah Definition: A process that converts synaptic vesicles to a state of competence for calcium triggered fusion with the active zone membrane by bringing the two membranes into very close proximity. Priming typically (but not always) occurs after docking (Jahn and Fasshauer, 2012). Primed vesicles are also capable of spontaneously fusing with the active zone membrane.